{
  "term_label": "cell migration",
  "gene_name": "Dedicator of cytokinesis protein 2",
  "term_id": "GO:0016477",
  "gene_symbol": "DOCK2",
  "gene": "UniProtKB:Q92608"
}